{
  "gene": "UniProtKB:Q14184",
  "gene_symbol": "DOC2B",
  "term_id": "GO:0045956",
  "gene_name": "Double C2-like domain-containing protein beta",
  "term_label": "positive regulation of calcium ion-dependent exocytosis"
}